{
  "gene": "UniProtKB:Q9BQS6",
  "gene_symbol": "HSPB9",
  "term_id": "GO:0005737",
  "term_label": "cytoplasm",
  "gene_name": "Heat shock protein beta-9"
}